{
  "term_label": "entrainment of circadian clock by photoperiod",
  "term_id": "GO:0043153",
  "gene": "UniProtKB:O15534",
  "gene_symbol": "PER1",
  "gene_name": "Period circadian protein homolog 1"
}